{
  "gene_symbol": "TGM7",
  "gene": "UniProtKB:Q96PF1",
  "term_label": "peptide cross-linking",
  "term_id": "GO:0018149",
  "gene_name": "Protein-glutamine gamma-glutamyltransferase Z"
}